nitrite transport [GO:0015707] (biological process) Sources: GOC:krc Relationships: is a type of inorganic anion transport [GO:0015698]; is a type of nitrogen compound transport [GO:0071705] Definition: The directed movement of nitrite into, out of or within a cell, or between cells, by means of some agent such as a transporter or pore.